{
  "gene": "UniProtKB:Q7Z3Z4",
  "gene_symbol": "PIWIL4",
  "term_id": "GO:0007283",
  "term_label": "spermatogenesis",
  "gene_name": "Piwi-like protein 4"
}